{
  "term_id": "GO:0032486",
  "gene_name": "Rap guanine nucleotide exchange factor 2",
  "term_label": "Rap protein signal transduction",
  "gene_symbol": "RAPGEF2",
  "gene": "UniProtKB:Q9Y4G8"
}